{
  "gene_name": "Sentrin-specific protease 3",
  "term_id": "GO:0005634",
  "term_label": "nucleus",
  "gene_symbol": "SENP3",
  "gene": "UniProtKB:Q9H4L4"
}